{
  "gene": "UniProtKB:P30793",
  "gene_name": "GTP cyclohydrolase 1",
  "term_label": "tetrahydrobiopterin biosynthetic process",
  "gene_symbol": "GCH1",
  "term_id": "GO:0006729"
}